{
  "gene": "UniProtKB:Q9NSD5",
  "term_label": "gamma-aminobutyric acid:sodium:chloride symporter activity",
  "term_id": "GO:0005332",
  "gene_symbol": "SLC6A13",
  "gene_name": "Sodium- and chloride-dependent GABA transporter 2"
}